2,3-dihydroxyindole 2,3-dioxygenase activity [GO:0047528] (molecular function) Sources: EC:1.13.11.23, RHEA:19445 Relationships: is a type of oxidoreductase activity, acting on single donors with incorporation of molecular oxygen, incorporation of two atoms of oxygen [GO:0016702] Definition: Catalysis of the reaction: 2,3-dihydroxyindole + O2 = anthranilate + CO2 + H+. Also known as: 2,3-dihydroxyindole:oxygen 2,3-oxidoreductase (decyclizing) activity